{
  "gene_symbol": "CD36",
  "gene": "UniProtKB:P16671",
  "term_id": "GO:0030169",
  "gene_name": "Platelet glycoprotein 4",
  "term_label": "low-density lipoprotein particle binding"
}